{
  "term_label": "phagocytosis",
  "gene_symbol": "MERTK",
  "gene": "UniProtKB:Q12866",
  "gene_name": "Tyrosine-protein kinase Mer",
  "term_id": "GO:0006909"
}